{
  "gene": "UniProtKB:P27930",
  "term_label": "cell surface",
  "term_id": "GO:0009986",
  "gene_name": "Interleukin-1 receptor type 2",
  "gene_symbol": "IL1R2"
}